{
  "term_id": "GO:0005737",
  "gene": "UniProtKB:Q8IU85",
  "gene_name": "Calcium_calmodulin-dependent protein kinase type 1D",
  "gene_symbol": "CAMK1D",
  "term_label": "cytoplasm"
}